{
  "term_label": "T cell receptor signaling pathway",
  "gene": "UniProtKB:P42681",
  "gene_name": "Tyrosine-protein kinase TXK",
  "gene_symbol": "TXK",
  "term_id": "GO:0050852"
}